{
  "gene": "UniProtKB:Q9ULB4",
  "term_id": "GO:0007043",
  "term_label": "cell-cell junction assembly",
  "gene_symbol": "CDH9",
  "gene_name": "Cadherin-9"
}